tRNA (cytidine(56)-2'-O)-methyltransferase activity [GO:0106059] (molecular function) Also known as: tRNA (cytidine 56-2'-O)-methyltransferase activity Relationships: is_a GO:0016427 Definition: Catalysis of the reaction: S-adenosyl-L-methionine + cytidine56 in tRNA= S-adenosyl-L-homocysteine + 2'-O-methylcytidine56 in tRNA. Sources: RHEA:42968